{
  "gene_name": "Putative serine_threonine-protein phosphatase 4 regulatory subunit 1-like",
  "term_label": "Unknown cellular component",
  "term_id": "UNKNOWN:0003",
  "gene": "UniProtKB:Q9P1A2",
  "gene_symbol": "PPP4R1L"
}